{
  "gene_symbol": "CLEC14A",
  "term_label": "extracellular matrix protein binding",
  "term_id": "GO:1990430",
  "gene_name": "C-type lectin domain family 14 member A",
  "gene": "UniProtKB:Q86T13"
}